{
  "gene_symbol": "SLC9C1",
  "term_id": "GO:0051453",
  "gene_name": "Sodium_hydrogen exchanger 10",
  "term_label": "regulation of intracellular pH",
  "gene": "UniProtKB:Q4G0N8"
}